neurotransmitter uptake [GO:0001504] (biological process) Regulation: regulated by regulation of neurotransmitter uptake [GO:0051580]; negatively regulated by negative regulation of neurotransmitter uptake [GO:0051581]; positively regulated by positive regulation of neurotransmitter uptake [GO:0051582] Subtypes: GO:0051615, neurotransmitter reuptake [GO:0098810] Definition: The directed movement of neurotransmitters into neurons or glial cells. This process leads to inactivation and recycling of neurotransmitters. Relationships: is a type of neurotransmitter transport [GO:0006836]; is a type of import into cell [GO:0098657] Also known as: neurotransmitter recycling, neurotransmitter import, neurotransmitter import into glial cell, neurotransmitter import into neuron Sources: ISBN:0123668387